{
  "gene_name": "Heterogeneous nuclear ribonucleoprotein L-like",
  "term_id": "GO:0003729",
  "gene": "UniProtKB:Q8WVV9",
  "gene_symbol": "HNRNPLL",
  "term_label": "mRNA binding"
}